{
  "term_id": "GO:0061844",
  "term_label": "antimicrobial humoral immune response mediated by antimicrobial peptide",
  "gene": "UniProtKB:Q16663",
  "gene_name": "C-C motif chemokine 15",
  "gene_symbol": "CCL15"
}